{
  "term_id": "GO:0035869",
  "term_label": "ciliary transition zone",
  "gene_name": "Transmembrane protein 17",
  "gene": "UniProtKB:Q86X19",
  "gene_symbol": "TMEM17"
}